{
  "term_label": "Unknown cellular component",
  "term_id": "UNKNOWN:0003",
  "gene_name": "Putative transmembrane protein encoded by LINC00862",
  "gene_symbol": "LINC00862",
  "gene": "UniProtKB:A6NCI5"
}